{
  "gene_symbol": "CLDN17",
  "gene_name": "Claudin-17",
  "gene": "UniProtKB:P56750",
  "term_id": "GO:0160187",
  "term_label": "paracellular tight junction channel activity"
}